{
  "gene_symbol": "VEGFC",
  "term_id": "GO:0050930",
  "gene_name": "Vascular endothelial growth factor C",
  "term_label": "induction of positive chemotaxis",
  "gene": "UniProtKB:P49767"
}